{
  "term_label": "phosphatidate phosphatase activity",
  "gene_name": "Phospholipid phosphatase 1",
  "term_id": "GO:0008195",
  "gene": "UniProtKB:O14494",
  "gene_symbol": "PLPP1"
}